{
  "term_id": "GO:0005929",
  "gene_symbol": "UNC119B",
  "gene_name": "Protein unc-119 homolog B",
  "term_label": "cilium",
  "gene": "UniProtKB:A6NIH7"
}